Fc receptor signaling pathway [GO:0038093] (biological process) Subtypes: Fc-gamma receptor signaling pathway [GO:0038094], GO:0038095 Sources: GOC:phg, Wikipedia:Fc_receptor Also known as: Fc receptor signalling pathway Definition: The series of molecular signals initiated by the binding of the Fc portion of an immunoglobulin to an Fc receptor on the surface of a target cell, and ending with the regulation of a downstream cellular process, e.g. transcription. The Fc portion of an immunoglobulin is its C-terminal constant region. Relationships: is a type of immune response-regulating cell surface receptor signaling pathway [GO:0002768]